mitochondrial RNA modification [GO:1900864] (biological process) Definition: Any RNA modification that takes place in mitochondrion. Sources: GOC:TermGenie Also known as: mitochondrial RNA editing Relationships: is a type of GO:0000959; is a type of RNA modification [GO:0009451] Subtypes: mitochondrial tRNA modification [GO:0070900], mitochondrial mRNA modification [GO:0080156]